i-AAA complex [GO:0031942] (cellular component) Relationships: is a type of inner mitochondrial membrane protein complex [GO:0098800] Definition: Protease complex of the mitochondrial inner membrane whose catalytic residues lie on the intermembrane space side of the inner membrane; involved in mitochondrial protein turnover. Contains a subunit belonging to the AAA family of ATP-dependent metalloproteases. References: PMID:16247555, PMID:16267274